{
  "gene_symbol": "VSIG10L2",
  "term_label": "cell-cell junction",
  "term_id": "GO:0005911",
  "gene": "UniProtKB:P0DP72",
  "gene_name": "V-set and immunoglobulin domain-containing protein 10-like 2"
}